retrograde trans-synaptic signaling [GO:0098917] (biological process) Sources: GOC:dos Definition: Cell-cell signaling from post to pre-synapse, across the synaptic cleft. Subtypes: retrograde trans-synaptic signaling by lipid [GO:0098920], GO:0098923, retrograde trans-synaptic signaling by trans-synaptic protein complex [GO:0098942], retrograde trans-synaptic signaling by neuropeptide [GO:0099082] Relationships: is a type of trans-synaptic signaling [GO:0099537]